{
  "gene": "UniProtKB:Q9UJU5",
  "gene_name": "Forkhead box protein D3",
  "term_label": "RNA polymerase II cis-regulatory region sequence-specific DNA binding",
  "term_id": "GO:0000978",
  "gene_symbol": "FOXD3"
}